vacuolar proton-transporting V-type ATPase, V0 domain [GO:0000220] (cellular component) Definition: The V0 domain of a proton-transporting V-type ATPase found in the vacuolar membrane. Relationships: is a type of proton-transporting V-type ATPase, V0 domain [GO:0033179]; is part of vacuolar proton-transporting V-type ATPase complex [GO:0016471] Note: Note that this domain often consists of five subunits, although in some mammalian tissues it may have an additional subunit. Subtypes: lysosomal proton-transporting V-type ATPase, V0 domain [GO:0046610] Also known as: vacuolar hydrogen ion-transporting ATPase V0 domain References: PMID:16449553 Sources: GOC:mah